{
  "term_id": "GO:0097400",
  "gene_name": "Interleukin-17A",
  "term_label": "interleukin-17-mediated signaling pathway",
  "gene_symbol": "IL17A",
  "gene": "UniProtKB:Q16552"
}